{
  "gene_name": "Phosphatidylinositol polyphosphate 5-phosphatase type IV",
  "gene": "UniProtKB:Q9NRR6",
  "term_label": "Golgi apparatus",
  "gene_symbol": "INPP5E",
  "term_id": "GO:0005794"
}